{
  "term_id": "GO:0038023",
  "gene_name": "Leucine-rich repeat-containing protein 17",
  "term_label": "signaling receptor activity",
  "gene": "UniProtKB:Q8N6Y2",
  "gene_symbol": "LRRC17"
}